{
  "term_label": "cytoplasmic vesicle",
  "gene_name": "Huntingtin",
  "gene_symbol": "HTT",
  "term_id": "GO:0031410",
  "gene": "UniProtKB:P42858"
}